{
  "gene_symbol": "CYP4A11",
  "gene_name": "Cytochrome P450 4A11",
  "term_label": "arachidonate metabolic process",
  "term_id": "GO:0019369",
  "gene": "UniProtKB:Q02928"
}